galactosidase activity [GO:0015925] (molecular function) Relationships: is a type of hydrolase activity, hydrolyzing O-glycosyl compounds [GO:0004553] Definition: Catalysis of the hydrolysis of galactosyl compounds, substances containing a group derived from a cyclic form of galactose or a galactose derivative. Subtypes: alpha-galactosidase activity [GO:0004557], beta-galactosidase activity [GO:0004565], arabinogalactan endo-1,4-beta-galactosidase activity [GO:0031218], GO:0033920, capsular-polysaccharide endo-1,3-alpha-galactosidase activity [GO:0033921], GO:0033929, keratan-sulfate endo-1,4-beta-galactosidase activity [GO:0033930] Sources: GOC:ai